{
  "gene": "UniProtKB:Q6P589",
  "term_id": "GO:0050868",
  "gene_name": "Tumor necrosis factor alpha-induced protein 8-like protein 2",
  "gene_symbol": "TNFAIP8L2",
  "term_label": "negative regulation of T cell activation"
}